{
  "gene": "UniProtKB:Q9NRA1",
  "term_label": "platelet-derived growth factor receptor signaling pathway",
  "gene_symbol": "PDGFC",
  "term_id": "GO:0048008",
  "gene_name": "Platelet-derived growth factor C"
}